{
  "term_id": "GO:0016538",
  "gene": "UniProtKB:Q96S94",
  "term_label": "cyclin-dependent protein serine/threonine kinase regulator activity",
  "gene_symbol": "CCNL2",
  "gene_name": "Cyclin-L2"
}